proton export across plasma membrane [GO:0120029] (biological process) Relationships: is a type of export across plasma membrane [GO:0140115]; is a type of proton transmembrane transport [GO:1902600] Also known as: hydrogen ion export from cell, proton export from cell, hydrogen ion export across plasma membrane Definition: The directed movement of hydrogen ions (protons) from inside a cell, across the plasma membrane and into the extracellular region. References: PMID:9762918 Sources: GOC:mah